B cell receptor transport into immunological synapse [GO:0032598] (biological process) Relationships: is a type of GO:0032597 Definition: The directed movement of a B cell receptor into an immunological synapse. Sources: GOC:mah Also known as: B cell receptor translocation into immunological synapse, BCR translocation into immunological synapse, BCR transport into immunological synapse